anterior lateral line neuromast cupula development [GO:0048904] (BP) Definition: The process whose specific outcome is the progression of the anterior lateral line neuromast cupula over time, from its formation to the mature structure. The cupula is secreted by mantle cells and the ciliary bundles of all of the hair cells of the neuromast are embedded in it. The cupula provides a mechanical linkage between the hair cells and the external hydrodynamic environment. The cupula of superficial neuromasts grows continuously, while the height of the cupula of canal neuromasts is limited by canal diameter. Sources: ISBN:0125296509 Relationships: is a type of cupula development [GO:0048887]; is part of anterior lateral line neuromast development [GO:0048901]